{
  "gene_symbol": "RPL34",
  "term_id": "GO:0003735",
  "term_label": "structural constituent of ribosome",
  "gene_name": "Large ribosomal subunit protein eL34",
  "gene": "UniProtKB:P49207"
}